T-helper 1 cell differentiation [GO:0045063] (biological process) Note: Note that immunologists typically use the word 'development' to refer to cells of B or T cell lineages undergoing the process that GO describes as 'cell differentiation'. Relationships: is a type of GO:0042093; is part of T-helper 1 type immune response [GO:0042088] Also known as: T-helper 1 cell development Sources: CL:0000545, GOC:ebc Definition: The process in which a relatively unspecialized T cell acquires the specialized features of a T-helper 1 (Th1) cell. A Th1 cell is a CD4-positive, alpha-beta T cell that has the phenotype T-bet-positive and produces interferon-gamma. Regulation: regulated by regulation of T-helper 1 cell differentiation [GO:0045625]; negatively regulated by negative regulation of T-helper 1 cell differentiation [GO:0045626]; positively regulated by positive regulation of T-helper 1 cell differentiation [GO:0045627]